{
  "term_id": "GO:0051016",
  "gene": "UniProtKB:Q13045",
  "gene_name": "Protein flightless-1 homolog",
  "gene_symbol": "FLII",
  "term_label": "barbed-end actin filament capping"
}